{
  "gene_symbol": "ATP9A",
  "gene": "UniProtKB:O75110",
  "term_label": "endosome",
  "term_id": "GO:0005768",
  "gene_name": "Probable phospholipid-transporting ATPase IIA"
}